regulation of exit from mitosis [GO:0007096] (biological process) Sources: GOC:rn Subtypes: negative regulation of exit from mitosis [GO:0001100], positive regulation of exit from mitosis [GO:0031536] Definition: Any process involved in the progression from anaphase/telophase to G1 that is associated with a conversion from high to low mitotic CDK activity. Relationships: is a type of regulation of mitotic cell cycle phase transition [GO:1901990]; regulates exit from mitosis [GO:0010458]